vomitoxin biosynthetic process [GO:0106110] (biological process) Relationships: is a type of sesquiterpenoid biosynthetic process [GO:0016106]; is a type of primary alcohol biosynthetic process [GO:0034309]; is a type of ketone biosynthetic process [GO:0042181]; is a type of mycotoxin biosynthetic process [GO:0043386]; is a type of polyol biosynthetic process [GO:0046173]; is a type of GO:0097176; is a type of GO:0120255; is a type of ether biosynthetic process [GO:1901503]; is a type of secondary alcohol biosynthetic process [GO:1902653] Also known as: DON biosynthetic process, deoxynivalenol biosynthetic process, vomitoxin anabolism, vomitoxin biosynthesis, vomitoxin formation, vomitoxin synthesis Definition: The chemical reactions and pathways resulting in the formation of type B trichothecene vomitoxin, also known as deoxynivalenol, a poisonous substance produced by some species of fungi and predominantly occurs in grains such as wheat, barley and oats. References: PMID:19333439, PMID:25680507, PMID:25758923, PMID:8637056 Sources: https://doi.org/10.1007/BF03356188